membrane repolarization during Purkinje myocyte action potential [GO:0086051] (biological process) Definition: The process in which ions are transported across a membrane such that the Purkinje myocyte membrane potential changes in the direction from the positive membrane potential at the peak of the action potential towards the negative resting potential. Relationships: is a type of membrane repolarization during cardiac muscle cell action potential [GO:0086013]; is part of Purkinje myocyte action potential [GO:0086017] Sources: GOC:BHF, GOC:dph, GOC:mtg_cardiac_conduct_nov11